{
  "term_label": "RNA helicase activity",
  "gene_symbol": "UPF1",
  "term_id": "GO:0003724",
  "gene_name": "Regulator of nonsense transcripts 1",
  "gene": "UniProtKB:Q92900"
}